{
  "gene": "UniProtKB:Q8IUM7",
  "gene_name": "Neuronal PAS domain-containing protein 4",
  "term_id": "GO:0000977",
  "gene_symbol": "NPAS4",
  "term_label": "RNA polymerase II transcription regulatory region sequence-specific DNA binding"
}